{
  "gene_name": "Zinc finger and BTB domain-containing protein 45",
  "term_label": "regulation of cytokine production",
  "term_id": "GO:0001817",
  "gene": "UniProtKB:Q96K62",
  "gene_symbol": "ZBTB45"
}